tachykinin receptor binding [GO:0071861] (molecular function) Sources: GOC:kmv, GOC:mah Definition: Binding to a tachykinin receptor. Relationships: is a type of neuropeptide receptor binding [GO:0071855]